{
  "gene_symbol": "C5orf22",
  "term_id": "UNKNOWN:0002",
  "gene": "UniProtKB:Q49AR2",
  "gene_name": "UPF0489 protein C5orf22",
  "term_label": "Unknown biological process"
}